{
  "gene_symbol": "FANCB",
  "term_label": "replication-born double-strand break repair via sister chromatid exchange",
  "term_id": "GO:1990414",
  "gene_name": "Fanconi anemia group B protein",
  "gene": "UniProtKB:Q8NB91"
}